{
  "term_id": "UNKNOWN:0003",
  "gene_symbol": "HSD17B8",
  "term_label": "Unknown cellular component",
  "gene": "UniProtKB:Q92506",
  "gene_name": "(3R)-3-hydroxyacyl-CoA dehydrogenase"
}